{
  "gene_name": "Rho GTPase-activating protein 17",
  "gene_symbol": "ARHGAP17",
  "term_label": "regulation of Rac protein signal transduction",
  "term_id": "GO:0035020",
  "gene": "UniProtKB:Q68EM7"
}